epithelial cell apoptotic process involved in palatal shelf morphogenesis [GO:1990134] (biological process) Relationships: is a type of apoptotic process involved in morphogenesis [GO:0060561]; is a type of epithelial cell apoptotic process [GO:1904019]; is part of GO:0062009 References: PMID:16607638 Sources: GOC:dph, GOC:mtg_apoptosis Definition: An apoptotic process in a palatal shelf epithelial cell that contributes to the shaping of the palatal shelf.